{
  "gene_symbol": "GRID1",
  "term_label": "modulation of chemical synaptic transmission",
  "gene_name": "Glutamate receptor ionotropic, delta-1",
  "gene": "UniProtKB:Q9ULK0",
  "term_id": "GO:0050804"
}